indole-3-acetonitrile nitrilase activity [GO:0080061] (molecular function) Relationships: is a type of GO:0000257 Sources: RHEA:45776 Definition: Catalysis of the reaction: indole-3-acetonitrile + 2 H2O = indole-3-acetic acid + NH3.